purine ribonucleoside diphosphate catabolic process [GO:0009181] (biological process) Definition: The chemical reactions and pathways resulting in the breakdown of purine ribonucleoside diphosphate, a compound consisting of a purine base linked to a ribose sugar esterified with diphosphate on the sugar. Sources: GOC:go_curators, ISBN:0198506732 Also known as: purine ribonucleoside diphosphate breakdown, purine ribonucleoside diphosphate catabolism, purine ribonucleoside diphosphate degradation Relationships: is a type of purine nucleoside diphosphate catabolic process [GO:0009137]; is a type of purine ribonucleoside diphosphate metabolic process [GO:0009179]; is a type of ribonucleoside diphosphate catabolic process [GO:0009191] Subtypes: ADP catabolic process [GO:0046032], IDP catabolic process [GO:0046709], GDP catabolic process [GO:0046712]